{
  "term_label": "Unknown cellular component",
  "gene_symbol": "SASH1",
  "term_id": "UNKNOWN:0003",
  "gene": "UniProtKB:O94885",
  "gene_name": "SAM and SH3 domain-containing protein 1"
}